epithelial cell maturation [GO:0002070] (biological process) Subtypes: columnar/cuboidal epithelial cell maturation [GO:0002069], epithelial cell maturation involved in salivary gland development [GO:0060691], epithelial cell maturation involved in prostate gland development [GO:0060743], GO:0072560 Sources: GOC:dph Relationships: is a type of GO:0048469; is part of epithelial cell development [GO:0002064] Definition: The developmental process, independent of morphogenetic (shape) change, that is required for an epithelial cell to attain its fully functional state. An epithelial cell is a cell usually found in a two-dimensional sheet with a free surface.